{
  "gene_name": "Failed axon connections homolog",
  "gene": "UniProtKB:Q5TGI0",
  "gene_symbol": "FAXC",
  "term_label": "Unknown cellular component",
  "term_id": "UNKNOWN:0003"
}